{
  "term_label": "axonemal microtubule",
  "term_id": "GO:0005879",
  "gene_symbol": "CFAP210",
  "gene": "UniProtKB:Q0VFZ6",
  "gene_name": "Cilia- and flagella- associated protein 210"
}